orcinol catabolic process [GO:0042209] (biological process) Also known as: orcin catabolic process, orcin catabolism, orcinol breakdown, orcinol catabolism, orcinol degradation Relationships: is a type of phenol-containing compound catabolic process [GO:0019336]; is a type of toluene-containing compound catabolic process [GO:0072491]; is_a GO:0090487 Definition: The chemical reactions and pathways resulting in the breakdown of orcinol (5-methyl-1,3-benzenediol), an aromatic compound derived from the fermentation of lichen and synthesized by some higher plants. Sources: GOC:jl